{
  "gene": "UniProtKB:P59901",
  "term_label": "cytokine-mediated signaling pathway",
  "gene_symbol": "LILRA4",
  "gene_name": "Leukocyte immunoglobulin-like receptor subfamily A member 4",
  "term_id": "GO:0019221"
}